{
  "gene_name": "Beta-adrenergic receptor kinase 2",
  "gene": "UniProtKB:P35626",
  "term_id": "GO:0002029",
  "term_label": "desensitization of G protein-coupled receptor signaling pathway",
  "gene_symbol": "GRK3"
}